{
  "term_id": "GO:0072393",
  "gene_name": "Protein bicaudal D homolog 2",
  "term_label": "microtubule anchoring at microtubule organizing center",
  "gene_symbol": "BICD2",
  "gene": "UniProtKB:Q8TD16"
}